{
  "term_id": "UNKNOWN:0003",
  "gene_name": "Protein ZNF767",
  "gene": "UniProtKB:Q75MW2",
  "gene_symbol": "ZNF767P",
  "term_label": "Unknown cellular component"
}